{
  "term_label": "DNA binding",
  "gene_symbol": "TIMELESS",
  "term_id": "GO:0003677",
  "gene_name": "Protein timeless homolog",
  "gene": "UniProtKB:Q9UNS1"
}